response to flavonoid [GO:1905395] (biological process) Subtypes: GO:1902168, response to quercetin [GO:1905235], GO:1905396 References: PMID:22700048 Sources: GOC:TermGenie, GO_REF:0000071 Definition: Any process that results in a change in state or activity of a cell or an organism (in terms of movement, secretion, enzyme production, gene expression, etc.) as a result of a flavonoid stimulus. Relationships: is a type of response to oxygen-containing compound [GO:1901700]